neuroblast fate commitment [GO:0014017] (biological process) Sources: GOC:ef, ISBN:0878932585 Definition: The process in which the developmental fate of a cell becomes restricted such that it will differentiate into a neuroblast. Relationships: is a type of GO:0045165; is part of GO:0014016 Subtypes: asymmetric neuroblast division resulting in ganglion mother cell formation [GO:0055060]